{
  "gene_symbol": "FLNC",
  "term_id": "UNKNOWN:0002",
  "gene": "UniProtKB:Q14315",
  "gene_name": "Filamin-C",
  "term_label": "Unknown biological process"
}